{
  "term_label": "Golgi organization",
  "gene_name": "Vacuole membrane protein 1",
  "gene_symbol": "VMP1",
  "term_id": "GO:0007030",
  "gene": "UniProtKB:Q96GC9"
}